{
  "term_id": "GO:0005634",
  "gene_name": "Cyclin-dependent kinase 8",
  "gene_symbol": "CDK8",
  "gene": "UniProtKB:P49336",
  "term_label": "nucleus"
}